regulation of demethylkotanin biosynthetic process [GO:1900652] (biological process) Also known as: regulation of demethylkotanin anabolism, regulation of demethylkotanin biosynthesis, regulation of demethylkotanin formation, regulation of demethylkotanin synthesis Relationships: is a type of GO:1900376; regulates demethylkotanin biosynthetic process [GO:1900599] Sources: GOC:TermGenie, GOC:di Definition: Any process that modulates the frequency, rate or extent of demethylkotanin biosynthetic process. Subtypes: negative regulation of demethylkotanin biosynthetic process [GO:1900653], GO:1900654